histamine transport [GO:0051608] (biological process) Sources: GOC:ai Definition: The directed movement of histamine into, out of or within a cell, or between cells, by means of some agent such as a transporter or pore. Histamine is a physiologically active amine, found in plant and animal tissue and released from mast cells as part of an allergic reaction in humans. Subtypes: histamine secretion [GO:0001821], histamine uptake [GO:0051615] Relationships: is a type of nitrogen compound transport [GO:0071705]